{
  "term_id": "GO:0030311",
  "term_label": "poly-N-acetyllactosamine biosynthetic process",
  "gene": "UniProtKB:Q6ZMB0",
  "gene_name": "Acetylgalactosaminyl-O-glycosyl-glycoprotein beta-1,3-N-acetylglucosaminyltransferase",
  "gene_symbol": "B3GNT6"
}